fumigaclavine C biosynthetic process [GO:1900809] (biological process) Definition: The chemical reactions and pathways resulting in the formation of fumigaclavine C, a fungal ergot alkaloid. Regulation: regulated by regulation of fumigaclavine C biosynthetic process [GO:1900837]; negatively regulated by negative regulation of fumigaclavine C biosynthetic process [GO:1900838]; positively regulated by positive regulation of fumigaclavine C biosynthetic process [GO:1900839] Relationships: is_a ergot alkaloid biosynthetic process [GO:0035837] Also known as: fumigaclavine C metabolic process, fumigaclavine C metabolism, fumigaclavine C anabolism, fumigaclavine C biosynthesis, fumigaclavine C formation, fumigaclavine C synthesis References: PMID:15933009, PMID:23435153, PMID:26972831 Sources: GOC:TermGenie, GOC:di